regulation of interferon-alpha production [GO:0032647] (biological process) Relationships: is a type of regulation of type I interferon production [GO:0032479]; regulates interferon-alpha production [GO:0032607] Subtypes: negative regulation of interferon-alpha production [GO:0032687], positive regulation of interferon-alpha production [GO:0032727] Definition: Any process that modulates the frequency, rate, or extent of interferon-alpha production. References: PMID:15546383 Sources: GOC:mah Also known as: regulation of interferon-alpha biosynthetic process, regulation of interferon-alpha secretion